lipooligosaccharide biosynthetic process [GO:1901271] (biological process) Sources: GOC:TermGenie, GOC:yaf, UniPathway:UPA00501 Subtypes: lipid A biosynthetic process [GO:0009245], Kdo2-lipid A biosynthetic process [GO:0036104], beta-L-Ara4N-lipid A biosynthetic process [GO:1901760] Relationships: is_a GO:1901137; is a type of lipooligosaccharide metabolic process [GO:1901269] Also known as: lipooligosaccharide anabolism, lipooligosaccharide biosynthesis, lipooligosaccharide formation, lipooligosaccharide synthesis Definition: The chemical reactions and pathways resulting in the formation of lipooligosaccharide.